{
  "term_id": "GO:0031012",
  "gene_symbol": "FBLN7",
  "gene": "UniProtKB:Q53RD9",
  "gene_name": "Fibulin-7",
  "term_label": "extracellular matrix"
}